glucan 1,4-alpha-maltotetraohydrolase activity [GO:0033910] (molecular function) Also known as: 1,4-alpha-D-glucan maltotetraohydrolase activity, G4-amylase activity, exo-maltotetraohydrolase activity, glucan 1,4-alpha-maltotetrahydrolase activity, maltotetraose-forming amylase activity Sources: EC:3.2.1.60 Definition: Catalysis of the hydrolysis of (1->4)-alpha-D-glucosidic linkages in amylaceous polysaccharides, to remove successive maltotetraose residues from the non-reducing chain ends. Relationships: is a type of GO:0004553